hermaphrodite germ-line sex determination [GO:0040021] (biological process) Relationships: is a type of GO:0018992 Sources: GOC:ems Subtypes: feminization of hermaphroditic germ-line [GO:0040022], masculinization of hermaphroditic germ-line [GO:0042006] Definition: The determination of sex and sexual phenotype in the germ line of a hermaphrodite.